{
  "gene_symbol": "LCP1",
  "term_label": "actin filament binding",
  "gene": "UniProtKB:P13796",
  "gene_name": "Plastin-2",
  "term_id": "GO:0051015"
}